{
  "term_id": "GO:0034375",
  "term_label": "high-density lipoprotein particle remodeling",
  "gene_name": "Pancreatic lipase-related protein 2",
  "gene_symbol": "PNLIPRP2",
  "gene": "UniProtKB:P54317"
}